{
  "gene_name": "Proenkephalin-B",
  "gene": "UniProtKB:P01213",
  "term_id": "GO:0030425",
  "gene_symbol": "PDYN",
  "term_label": "dendrite"
}